{
  "gene_symbol": "Q6ZRN7",
  "gene_name": "Putative uncharacterized protein FLJ46214",
  "term_id": "UNKNOWN:0001",
  "gene": "UniProtKB:Q6ZRN7",
  "term_label": "Unknown molecular function"
}